{
  "gene_name": "Vasorin",
  "term_label": "plasma membrane",
  "gene_symbol": "VASN",
  "term_id": "GO:0005886",
  "gene": "UniProtKB:Q6EMK4"
}